{
  "gene": "UniProtKB:Q8WV19",
  "gene_symbol": "SFT2D1",
  "term_label": "Unknown cellular component",
  "gene_name": "Vesicle transport protein SFT2A",
  "term_id": "UNKNOWN:0003"
}